{
  "term_id": "GO:0005634",
  "gene_name": "Zinc finger protein 836",
  "term_label": "nucleus",
  "gene_symbol": "ZNF836",
  "gene": "UniProtKB:Q6ZNA1"
}